{
  "term_label": "minus-end-directed microtubule motor activity",
  "gene_name": "Dynein axonemal heavy chain 8",
  "gene": "UniProtKB:Q96JB1",
  "term_id": "GO:0008569",
  "gene_symbol": "DNAH8"
}